{
  "term_label": "cytoplasm",
  "gene": "UniProtKB:Q9GZT8",
  "term_id": "GO:0005737",
  "gene_symbol": "NIF3L1",
  "gene_name": "NIF3-like protein 1"
}